membrane insertase activity [GO:0032977] (molecular function) References: PMID:14739936, PMID:29809151, PMID:30415835, PMID:32459176 Definition: Binds transmembrane domain-containing proteins and mediates their integration into a membrane. Relationships: is a type of protein carrier chaperone [GO:0140597]; is part of establishment of protein localization to membrane [GO:0090150]